{
  "term_id": "GO:0005096",
  "gene": "UniProtKB:A1A4S6",
  "gene_name": "Rho GTPase-activating protein 10",
  "gene_symbol": "ARHGAP10",
  "term_label": "GTPase activator activity"
}